{
  "term_id": "GO:0001682",
  "term_label": "tRNA 5'-leader removal",
  "gene": "UniProtKB:O95059",
  "gene_symbol": "RPP14",
  "gene_name": "Ribonuclease P protein subunit p14"
}